telomeric G-quadruplex DNA binding [GO:0061849] (molecular function) References: PMID:16142245, PMID:9512530 Sources: GOC:BHF, GOC:BHF_telomere, GOC:nc Definition: Binding to telomeric G-quadruplex DNA structures, in which groups of four guanines adopt a flat, cyclic Hoogsteen hydrogen-bonding arrangement known as a guanine tetrad. The stacking of guanine tetrads results in G-quadruplex DNA structures in telomeres. Relationships: is a type of telomeric DNA binding [GO:0042162]; is a type of G-quadruplex DNA binding [GO:0051880]